{
  "gene_name": "Deleted in azoospermia protein 1",
  "term_id": "GO:0045948",
  "gene_symbol": "DAZ1",
  "gene": "UniProtKB:Q9NQZ3",
  "term_label": "positive regulation of translational initiation"
}